{
  "term_label": "protein ubiquitination",
  "gene_name": "Cullin-2",
  "term_id": "GO:0016567",
  "gene": "UniProtKB:Q13617",
  "gene_symbol": "CUL2"
}